{
  "gene_name": "Mitochondrial 10-formyltetrahydrofolate dehydrogenase",
  "term_label": "Unknown biological process",
  "gene": "UniProtKB:Q3SY69",
  "term_id": "UNKNOWN:0002",
  "gene_symbol": "ALDH1L2"
}